rhythmic process [GO:0048511] (biological process) Definition: Any process pertinent to the generation and maintenance of rhythms in the physiology of an organism. Relationships: is a type of biological_process [GO:0008150] Subtypes: circadian rhythm [GO:0007623], ultradian rhythm [GO:0007624], ovulation cycle process [GO:0022602], GO:0042698 Also known as: rhythm Sources: GOC:jid